{
  "gene_name": "Keratin, type I cytoskeletal 25",
  "gene": "UniProtKB:Q7Z3Z0",
  "term_label": "structural constituent of skin epidermis",
  "gene_symbol": "KRT25",
  "term_id": "GO:0030280"
}